cytospinule [GO:0160231] (cellular component) References: PMID:28490731, PMID:37863104 Relationships: is a type of GO:0098858 Definition: An actin-based cell projection extending laterally from the basolateral membrane of tuft cells in epithelial tissues, including the intestinal epithelium. These thin projections, typically 3-4 per cell and up to 3 micron long, directly contact the nuclei of adjacent epithelial cells, potentially facilitating intercellular communication and molecular exchange.